{
  "term_id": "GO:0048019",
  "term_label": "receptor antagonist activity",
  "gene_symbol": "MTRNR2L8",
  "gene_name": "Humanin-like 8",
  "gene": "UniProtKB:P0CJ75"
}